{
  "term_id": "GO:0005634",
  "gene_symbol": "IPPK",
  "gene": "UniProtKB:Q9H8X2",
  "gene_name": "Inositol-pentakisphosphate 2-kinase",
  "term_label": "nucleus"
}